{
  "gene": "UniProtKB:Q06250",
  "gene_symbol": "WT1-AS",
  "gene_name": "Putative Wilms tumor upstream neighbor 1 gene protein",
  "term_id": "UNKNOWN:0001",
  "term_label": "Unknown molecular function"
}